{
  "term_id": "UNKNOWN:0001",
  "gene_name": "Ensconsin",
  "gene_symbol": "MAP7",
  "gene": "UniProtKB:Q14244",
  "term_label": "Unknown molecular function"
}